{
  "gene_symbol": "SUSD6",
  "term_id": "UNKNOWN:0003",
  "gene": "UniProtKB:Q92537",
  "gene_name": "Sushi domain-containing protein 6",
  "term_label": "Unknown cellular component"
}